{
  "gene": "UniProtKB:Q5NDL2",
  "term_id": "GO:0097363",
  "term_label": "protein O-acetylglucosaminyltransferase activity",
  "gene_symbol": "EOGT",
  "gene_name": "EGF domain-specific O-linked N-acetylglucosamine transferase"
}